positive regulation of plasma cell differentiation [GO:1900100] (biological process) Definition: Any process that activates or increases the frequency, rate or extent of plasma cell differentiation. Sources: GOC:TermGenie Also known as: up regulation of plasma cell differentiation, up-regulation of plasma cell differentiation, upregulation of plasma cell differentiation, activation of plasma cell differentiation, activation of plasma cell development, positive regulation of plasma cell development, up regulation of plasma cell development, up-regulation of plasma cell development, upregulation of plasma cell development Relationships: is a type of positive regulation of immune effector process [GO:0002699]; is a type of positive regulation of B cell differentiation [GO:0045579]; is a type of positive regulation of immune response [GO:0050778]; is a type of GO:1900098; positively regulates plasma cell differentiation [GO:0002317]